{
  "gene_symbol": "ZNF366",
  "term_id": "GO:0003700",
  "gene": "UniProtKB:Q8N895",
  "term_label": "DNA-binding transcription factor activity",
  "gene_name": "Zinc finger protein 366"
}